{
  "term_label": "proteasome assembly",
  "gene": "UniProtKB:Q9Y244",
  "term_id": "GO:0043248",
  "gene_symbol": "POMP",
  "gene_name": "Proteasome maturation protein"
}